{
  "gene_name": "Cadherin-20",
  "gene": "UniProtKB:Q9HBT6",
  "term_id": "GO:0044331",
  "term_label": "cell-cell adhesion mediated by cadherin",
  "gene_symbol": "CDH20"
}